(3S)-3-hydroxyacyl-CoA dehydrogenase (NAD+) activity [GO:0003857] (molecular function) Definition: Catalysis of the reaction: a (3S)-3-hydroxyacyl-CoA + NAD+ = a 3-oxoacyl-CoA + NADH + H+. Sources: RHEA:22432 Relationships: is a type of GO:0016616 Also known as: beta-ketoacyl-CoA reductase, beta-hydroxybutyrylcoenzyme A dehydrogenase activity, 3-oxoacyl-thioester reductase activity, L-3-hydroxyacyl CoA dehydrogenase activity, L-3-hydroxyacyl coenzyme A dehydrogenase activity, beta-hydroxyacyl dehydrogenase activity, beta-hydroxyacyl-coenzyme A synthetase activity, beta-hydroxyacylcoenzyme A dehydrogenase activity, beta-keto-reductase activity Subtypes: long-chain (3S)-3-hydroxyacyl-CoA dehydrogenase (NAD+) activity [GO:0016509]